{
  "gene_symbol": "ABHD13",
  "gene_name": "Protein ABHD13",
  "gene": "UniProtKB:Q7L211",
  "term_id": "UNKNOWN:0002",
  "term_label": "Unknown biological process"
}